{
  "term_label": "Unknown cellular component",
  "term_id": "UNKNOWN:0003",
  "gene_symbol": "FUT2",
  "gene": "UniProtKB:Q10981",
  "gene_name": "Galactoside alpha-(1,2)-fucosyltransferase 2"
}